protein-lysine N-methyltransferase activity [GO:0016279] (molecular function) Definition: Catalysis of the transfer of a methyl group from S-adenosyl-L-methionine to the epsilon-amino group of a lysine residue in a protein substrate. Relationships: is a type of protein methyltransferase activity [GO:0008276]; is a type of lysine N-methyltransferase activity [GO:0016278] Subtypes: [cytochrome c]-lysine N-methyltransferase activity [GO:0000277], calmodulin-lysine N-methyltransferase activity [GO:0018025], histone H3K79 methyltransferase activity [GO:0031151], histone H4K20 methyltransferase activity [GO:0042799], histone H3K4 methyltransferase activity [GO:0042800], histone H3K9 methyltransferase activity [GO:0046974], histone H3K36 methyltransferase activity [GO:0046975], histone H3K27 methyltransferase activity [GO:0046976], histone H3K37 methyltransferase activity [GO:0062122], histone H3K56 methyltransferase activity [GO:0140759], histone H4K12 methyltransferase activity [GO:0140984] Also known as: protein (lysine) methyltransferase activity, protein lysine methylase activity References: PMID:12054878